{
  "term_label": "phosphatidylinositol-3,5-bisphosphate 3-phosphatase activity",
  "gene_symbol": "MTMR4",
  "gene_name": "Myotubularin-related protein 4",
  "term_id": "GO:0052629",
  "gene": "UniProtKB:Q9NYA4"
}